{
  "term_id": "GO:0015031",
  "gene_name": "Charged multivesicular body protein 3",
  "gene_symbol": "CHMP3",
  "term_label": "protein transport",
  "gene": "UniProtKB:Q9Y3E7"
}